{
  "gene": "UniProtKB:Q8TCB7",
  "term_id": "UNKNOWN:0003",
  "term_label": "Unknown cellular component",
  "gene_name": "tRNA N(3)-methylcytidine methyltransferase METTL6",
  "gene_symbol": "METTL6"
}